{
  "term_label": "Unknown biological process",
  "term_id": "UNKNOWN:0002",
  "gene_name": "Beta-defensin 112",
  "gene": "UniProtKB:Q30KQ8",
  "gene_symbol": "DEFB112"
}